{
  "gene_symbol": "CD1C",
  "term_label": "immune response",
  "gene_name": "T-cell surface glycoprotein CD1c",
  "gene": "UniProtKB:P29017",
  "term_id": "GO:0006955"
}